{
  "gene_symbol": "TXNDC17",
  "gene": "UniProtKB:Q9BRA2",
  "term_label": "Unknown biological process",
  "term_id": "UNKNOWN:0002",
  "gene_name": "Thioredoxin domain-containing protein 17"
}